{
  "term_id": "UNKNOWN:0001",
  "gene": "UniProtKB:A0A2R8Y4Y8",
  "gene_symbol": "OOSP4B",
  "term_label": "Unknown molecular function",
  "gene_name": "Oocyte-secreted protein 4B"
}